{
  "term_id": "GO:0010669",
  "term_label": "epithelial structure maintenance",
  "gene_name": "FRAS1-related extracellular matrix protein 2",
  "gene_symbol": "FREM2",
  "gene": "UniProtKB:Q5SZK8"
}